heptaprenylglyceryl phosphate synthase activity [GO:0120536] (molecular function) References: PMID:21761520 Sources: RHEA:33495 Definition: Catalysis of the reaction: sn-glycerol 1-phosphate + all-trans-heptaprenyl diphosphate = 3-heptaprenyl-sn-glycero-1-phosphate + diphosphate. Also known as: HepGP synthase activity, glycerol-1-phosphate heptaprenyltransferase activity Relationships: is a type of prenyltransferase activity [GO:0004659]